{
  "gene_name": "Coiled-coil domain-containing protein 181",
  "gene": "UniProtKB:Q5TID7",
  "gene_symbol": "CCDC181",
  "term_label": "Unknown cellular component",
  "term_id": "UNKNOWN:0003"
}